{
  "gene_name": "Membrane primary amine oxidase",
  "term_label": "early endosome",
  "gene_symbol": "AOC3",
  "term_id": "GO:0005769",
  "gene": "UniProtKB:Q16853"
}